negative regulation of gap junction assembly [GO:1903597] (biological process) References: PMID:25017399 Sources: GOC:BHF, GOC:TermGenie, GOC:mtg_cardiac_conduct_nov11, GOC:rl, GO_REF:0000058 Also known as: down regulation of gap junction assembly, down-regulation of gap junction assembly, downregulation of gap junction assembly, inhibition of gap junction assembly Relationships: is a type of GO:1901889; is a type of GO:1903596; RO_0002212 gap junction assembly [GO:0016264] Definition: Any process that stops, prevents or reduces the frequency, rate or extent of gap junction assembly.